{
  "gene": "UniProtKB:Q14721",
  "term_id": "GO:0032809",
  "gene_name": "Potassium voltage-gated channel subfamily B member 1",
  "term_label": "neuronal cell body membrane",
  "gene_symbol": "KCNB1"
}